{
  "term_label": "mitochondrion",
  "term_id": "GO:0005739",
  "gene": "UniProtKB:P34896",
  "gene_name": "Serine hydroxymethyltransferase, cytosolic",
  "gene_symbol": "SHMT1"
}